small GTPase binding [GO:0031267] (molecular function) Also known as: ADP-ribosylation factor binding, ARF binding, GTP-Ral binding, GTP-Rho binding, REP, Rab GTPase binding, Rab escort protein activity, Rab interactor activity, Rac GTPase binding, Ral GTPase binding, Ran GTPase binding, Ran protein binding, Ran-binding protein, Ras GTPase binding, Ras interactor activity, Rho GTPase binding Relationships: is_a GTPase binding [GO:0051020] Definition: Binding to a small monomeric GTPase. References: PMID:27218782 Sources: GOC:mah